{
  "gene_symbol": "CYTL1",
  "gene": "UniProtKB:Q9NRR1",
  "term_label": "positive regulation of transcription by RNA polymerase II",
  "gene_name": "Cytokine-like protein 1",
  "term_id": "GO:0045944"
}